{
  "gene_name": "XK-related protein 3",
  "term_id": "UNKNOWN:0002",
  "term_label": "Unknown biological process",
  "gene": "UniProtKB:Q5GH77",
  "gene_symbol": "XKR3"
}